{
  "gene_symbol": "SOD3",
  "term_id": "GO:0004784",
  "gene_name": "Extracellular superoxide dismutase [Cu-Zn]",
  "term_label": "superoxide dismutase activity",
  "gene": "UniProtKB:P08294"
}